{
  "gene": "UniProtKB:Q9P2C4",
  "term_label": "Unknown cellular component",
  "gene_symbol": "TMEM181",
  "gene_name": "Transmembrane protein 181",
  "term_id": "UNKNOWN:0003"
}